{
  "term_id": "GO:0015910",
  "gene_symbol": "ABCD4",
  "gene_name": "Lysosomal cobalamin transporter ABCD4",
  "term_label": "long-chain fatty acid import into peroxisome",
  "gene": "UniProtKB:O14678"
}